{
  "term_id": "GO:0004888",
  "gene_symbol": "C17orf99",
  "gene_name": "Protein IL-40",
  "gene": "UniProtKB:Q6UX52",
  "term_label": "transmembrane signaling receptor activity"
}